{
  "term_id": "UNKNOWN:0001",
  "gene_symbol": "LINC01555",
  "term_label": "Unknown molecular function",
  "gene_name": "Putative uncharacterized protein encoded by LINC01555",
  "gene": "UniProtKB:Q8NAE3"
}